{
  "term_label": "PML body",
  "term_id": "GO:0016605",
  "gene_name": "Calcium-binding and coiled-coil domain-containing protein 2",
  "gene": "UniProtKB:Q13137",
  "gene_symbol": "CALCOCO2"
}